{
  "term_id": "UNKNOWN:0001",
  "gene": "UniProtKB:E7EW31",
  "term_label": "Unknown molecular function",
  "gene_name": "Proline-rich basic protein 1",
  "gene_symbol": "PROB1"
}